trimethylamine dehydrogenase activity [GO:0050470] (MF) Sources: EC:1.5.8.2, MetaCyc:1.5.8.2-RXN Also known as: TMADh activity, trimethylamine:electron-transferring flavoprotein oxidoreductase (demethylating) Relationships: is a type of oxidoreductase activity, acting on the CH-NH group of donors, flavin as acceptor [GO:0046997] Definition: Catalysis of the reaction: trimethylamine + H2O + electron-transferring flavoprotein = dimethylamine + formaldehyde + reduced electron-transferring flavoprotein.